C-terminal protein deglutamylation [GO:0035609] (biological process) Relationships: is a type of C-terminal protein amino acid modification [GO:0018410]; is a type of protein deglutamylation [GO:0035608] Also known as: protein primary sequence deglutamylation References: PMID:21074048 Sources: GOC:sp Definition: The removal of a C-terminal, gene-encoded glutamate residue from a protein.